{
  "gene_symbol": "ABRAXAS1",
  "gene": "UniProtKB:Q6UWZ7",
  "term_id": "GO:0005634",
  "term_label": "nucleus",
  "gene_name": "BRCA1-A complex subunit Abraxas 1"
}